prostanoid metabolic process [GO:0006692] (biological process) Relationships: is a type of icosanoid metabolic process [GO:0006690]; is a type of GO:0033559 Definition: The chemical reactions and pathways involving prostanoids, any compound based on or derived from the prostanoate structure. Sources: ISBN:0198506732 Also known as: prostanoid metabolism Subtypes: prostaglandin metabolic process [GO:0006693], prostanoid biosynthetic process [GO:0046457]